{
  "gene_symbol": "SRPRB",
  "term_label": "signal recognition particle receptor complex",
  "gene_name": "Signal recognition particle receptor subunit beta",
  "gene": "UniProtKB:Q9Y5M8",
  "term_id": "GO:0005785"
}